{
  "term_label": "Unknown biological process",
  "gene_name": "Putative protein SPATA31F2P",
  "gene": "UniProtKB:Q63HN1",
  "gene_symbol": "SPATA31F2P",
  "term_id": "UNKNOWN:0002"
}